{
  "term_id": "UNKNOWN:0002",
  "gene": "UniProtKB:Q8WWQ8",
  "gene_name": "Stabilin-2",
  "term_label": "Unknown biological process",
  "gene_symbol": "STAB2"
}